{
  "gene_symbol": "FBXL12",
  "term_id": "GO:0031146",
  "term_label": "SCF-dependent proteasomal ubiquitin-dependent protein catabolic process",
  "gene_name": "F-box_LRR-repeat protein 12",
  "gene": "UniProtKB:Q9NXK8"
}